{
  "gene_symbol": "KIF27",
  "gene_name": "Kinesin-like protein KIF27",
  "gene": "UniProtKB:Q86VH2",
  "term_label": "kinesin complex",
  "term_id": "GO:0005871"
}